{
  "term_id": "GO:0004500",
  "gene_symbol": "DBH",
  "gene_name": "Dopamine beta-hydroxylase",
  "gene": "UniProtKB:P09172",
  "term_label": "dopamine beta-monooxygenase activity"
}